{
  "gene_name": "G-protein coupled receptor 161",
  "term_label": "recycling endosome",
  "gene_symbol": "GPR161",
  "term_id": "GO:0055037",
  "gene": "UniProtKB:Q8N6U8"
}